negative regulation of axon guidance [GO:1902668] (biological process) References: PMID:23006775 Sources: GOC:TermGenie, GOC:hjd, GO_REF:0000058 Relationships: is a type of negative regulation of neuron projection development [GO:0010977]; is a type of negative regulation of chemotaxis [GO:0050922]; is a type of regulation of axon guidance [GO:1902667]; negatively regulates axon guidance [GO:0007411] Also known as: down regulation of axon guidance, down regulation of axon pathfinding, down-regulation of axon guidance, down-regulation of axon pathfinding, downregulation of axon guidance, downregulation of axon pathfinding, negative regulation of axon pathfinding, down regulation of axon growth cone guidance, down-regulation of axon growth cone guidance, downregulation of axon growth cone guidance, inhibition of axon growth cone guidance, inhibition of axon guidance, inhibition of axon pathfinding, negative regulation of axon growth cone guidance, down regulation of axon chemotaxis, down-regulation of axon chemotaxis, downregulation of axon chemotaxis, inhibition of axon chemotaxis, negative regulation of axon chemotaxis Subtypes: GO:0090260, negative regulation of anterior/posterior axon guidance [GO:1905487], negative regulation of sensory neuron axon guidance [GO:1905490], GO:1905813, negative regulation of dorsal/ventral axon guidance [GO:1905816] Definition: Any process that stops, prevents or reduces the frequency, rate or extent of axon guidance.